positive regulation of methane biosynthetic process from carbon monoxide [GO:1900338] (biological process) Relationships: is a type of regulation of methane biosynthetic process from carbon monoxide [GO:1900336]; is a type of positive regulation of alkane biosynthetic process [GO:1901579]; is a type of positive regulation of cellular respiration [GO:1901857]; positively regulates methane biosynthetic process from carbon monoxide [GO:2001134] Also known as: up regulation of methane biosynthetic process from carbon monoxide, up-regulation of methane biosynthetic process from carbon monoxide, upregulation of methane biosynthetic process from carbon monoxide, activation of methane biosynthetic process from carbon monoxide Sources: GOC:TermGenie, GOC:mengo_curators Definition: Any process that activates or increases the frequency, rate or extent of methane biosynthetic process from carbon monoxide.